{
  "term_label": "structural constituent of ribosome",
  "gene": "UniProtKB:Q02543",
  "gene_name": "Large ribosomal subunit protein eL20",
  "gene_symbol": "RPL18A",
  "term_id": "GO:0003735"
}